{
  "term_id": "GO:0016491",
  "term_label": "oxidoreductase activity",
  "gene": "UniProtKB:P0C7P4",
  "gene_symbol": "UQCRFS1P1",
  "gene_name": "Putative cytochrome b-c1 complex subunit Rieske-like protein 1"
}